{
  "gene": "UniProtKB:Q9H5U6",
  "term_id": "GO:0008988",
  "gene_symbol": "ZCCHC4",
  "gene_name": "rRNA N6-adenosine-methyltransferase ZCCHC4",
  "term_label": "rRNA (adenine-N6-)-methyltransferase activity"
}